negative regulation of T cell mediated cytotoxicity [GO:0001915] (biological process) Sources: GOC:add, ISBN:0781735149 Definition: Any process that stops, prevents, or reduces the rate of T cell mediated cytotoxicity. Subtypes: GO:0002853, negative regulation of cytotoxic T cell degranulation [GO:0043318] Relationships: is a type of negative regulation of leukocyte mediated cytotoxicity [GO:0001911]; is a type of regulation of T cell mediated cytotoxicity [GO:0001914]; is a type of negative regulation of T cell mediated immunity [GO:0002710]; negatively regulates T cell mediated cytotoxicity [GO:0001913] Also known as: down regulation of T cell mediated cytotoxicity, down-regulation of T cell mediated cytotoxicity, downregulation of T cell mediated cytotoxicity, negative regulation of T cell mediated apoptosis, negative regulation of T cell mediated cell death, negative regulation of T cell mediated cell killing, negative regulation of T lymphocyte mediated cytotoxicity, negative regulation of T-cell mediated apoptosis, negative regulation of T-cell mediated cell death, negative regulation of T-cell mediated cell killing, negative regulation of T-cell mediated cytotoxicity, negative regulation of T-lymphocyte mediated cytotoxicity, inhibition of T cell mediated cytotoxicity, negative regulation of T cell mediated cytolysis, negative regulation of T-cell mediated cytolysis